{
  "term_label": "extracellular space",
  "term_id": "GO:0005615",
  "gene_symbol": "MUC6",
  "gene_name": "Mucin-6",
  "gene": "UniProtKB:Q6W4X9"
}